{
  "gene_name": "Grainyhead-like protein 3 homolog",
  "term_id": "GO:0001228",
  "gene_symbol": "GRHL3",
  "gene": "UniProtKB:Q8TE85",
  "term_label": "DNA-binding transcription activator activity, RNA polymerase II-specific"
}